fibrous body-membranous organelle [GO:0160208] (cellular component) Also known as: FB-MO Relationships: is a type of intracellular membrane-bounded organelle [GO:0043231] References: PMID:18050478, PMID:8004009 Definition: A Golgi-derived organelle that forms in primary spermatocytes during spermatogenesis of some nematodes including C. elegans. This 'double organelle' consists of a fibrous body containing major sperm protein and a membranous organelle that envelops the developing fibrous body.